{
  "gene_name": "Putative protein FAM90A22",
  "term_label": "Unknown molecular function",
  "gene": "UniProtKB:A8MWA6",
  "term_id": "UNKNOWN:0001",
  "gene_symbol": "FAM90A22"
}